negative regulation of activation of membrane attack complex [GO:0001971] (biological process) Definition: Any process that stops, prevents, or reduces the frequency, rate or extent of the activation of the membrane attack complex components of the complement cascade. Sources: GOC:hjd Relationships: is a type of GO:0001969; is a type of negative regulation of complement activation [GO:0045916]; negatively regulates activation of membrane attack complex [GO:0001905] Also known as: down regulation of activation of membrane attack complex, down-regulation of activation of membrane attack complex, downregulation of activation of membrane attack complex, negative regulation of MAC assembly, negative regulation of MAC formation, negative regulation of activation of MAC, negative regulation of membrane attack complex assembly, negative regulation of membrane attack complex formation, inhibition of activation of membrane attack complex, negative regulation of activation of TCC, negative regulation of activation of terminal complement complex, negative regulation of activation of the terminal complement cascade